lipoprotein particle mediated signaling [GO:0055095] (BP) Relationships: is a type of GO:0007165; is part of cellular response to lipoprotein particle stimulus [GO:0071402] Sources: GOC:BHF, GOC:rl Definition: The series of molecular signals mediated by the detection of a lipoprotein particle. Subtypes: low-density lipoprotein particle mediated signaling [GO:0055096], high density lipoprotein particle mediated signaling [GO:0055097] Also known as: lipoprotein mediated signalling, lipoprotein particle mediated signal transduction, lipoprotein particle-mediated signaling